auditory receptor cell morphogenesis [GO:0002093] (biological process) Definition: Any process that alters the size or shape of an auditory receptor cell. Also known as: hair cell morphogenesis Relationships: is a type of GO:0048598; is a type of cell morphogenesis involved in neuron differentiation [GO:0048667]; BFO_0000050 inner ear morphogenesis [GO:0042472]; is part of auditory receptor cell development [GO:0060117] Sources: GOC:dph, GOC:tb